carcinine transmembrane transporter activity [GO:1905131] (molecular function) Definition: Enables the transfer of carcinine from one side of a membrane to the other. Relationships: is a type of amide transmembrane transporter activity [GO:0042887]; is a type of modified amino acid transmembrane transporter activity [GO:0072349]; is a type of azole transmembrane transporter activity [GO:1901474] References: PMID:26653853, PMID:26713872 Sources: GOC:TermGenie, GOC:dph, GO_REF:0000070